{
  "gene_name": "Glucose-induced degradation protein 4 homolog",
  "term_label": "ubiquitin protein ligase activity",
  "term_id": "GO:0061630",
  "gene": "UniProtKB:Q8IVV7",
  "gene_symbol": "GID4"
}